{
  "term_label": "Unknown cellular component",
  "gene_name": "Uncharacterized protein encoded by LINC02872",
  "gene_symbol": "LINC02872",
  "gene": "UniProtKB:A2RU37",
  "term_id": "UNKNOWN:0003"
}